{
  "term_label": "Unknown cellular component",
  "gene_symbol": "MAB21L4",
  "gene_name": "Protein mab-21-like 4",
  "gene": "UniProtKB:Q08AI8",
  "term_id": "UNKNOWN:0003"
}